{
  "term_label": "plasma membrane",
  "term_id": "GO:0005886",
  "gene_name": "Immunoglobulin-like domain-containing receptor 1",
  "gene": "UniProtKB:Q86SU0",
  "gene_symbol": "ILDR1"
}